{
  "gene_symbol": "KIF5A",
  "term_label": "cytoplasm",
  "term_id": "GO:0005737",
  "gene": "UniProtKB:Q12840",
  "gene_name": "Kinesin heavy chain isoform 5A"
}